{
  "gene": "UniProtKB:Q6PEX7",
  "gene_symbol": "TEX38",
  "gene_name": "Testis-expressed protein 38",
  "term_label": "Unknown cellular component",
  "term_id": "UNKNOWN:0003"
}